{
  "term_label": "Unknown biological process",
  "gene_symbol": "RPL18",
  "gene_name": "Large ribosomal subunit protein eL18",
  "gene": "UniProtKB:Q07020",
  "term_id": "UNKNOWN:0002"
}